{
  "term_label": "9+2 motile cilium",
  "gene_symbol": "DNAH11",
  "gene_name": "Dynein axonemal heavy chain 11",
  "gene": "UniProtKB:Q96DT5",
  "term_id": "GO:0097729"
}